{
  "gene_symbol": "ESRRG",
  "gene_name": "Estrogen-related receptor gamma",
  "gene": "UniProtKB:P62508",
  "term_id": "GO:0034056",
  "term_label": "estrogen response element binding"
}